{
  "term_id": "GO:0034514",
  "gene_name": "60 kDa heat shock protein, mitochondrial",
  "gene_symbol": "HSPD1",
  "term_label": "mitochondrial unfolded protein response",
  "gene": "UniProtKB:P10809"
}